{
  "gene_symbol": "MCFD2",
  "gene": "UniProtKB:Q8NI22",
  "term_id": "UNKNOWN:0001",
  "gene_name": "Multiple coagulation factor deficiency protein 2",
  "term_label": "Unknown molecular function"
}